{
  "term_label": "endoplasmic reticulum membrane",
  "term_id": "GO:0005789",
  "gene_name": "Golgi SNAP receptor complex member 2",
  "gene": "UniProtKB:O14653",
  "gene_symbol": "GOSR2"
}